pore formation in membrane of another organism [GO:0035915] (BP) Definition: The aggregation, arrangement and bonding together of a set of components by an organism to form a pore complex in a membrane of another organism. Relationships: is a type of disruption of plasma membrane integrity in another organism [GO:0051673] References: PMID:21549739 Sources: GOC:bf, GOC:fj Also known as: pore complex assembly in other organism, pore complex biogenesis in other organism, pore formation in membrane of other organism, pore formation in other organism, pore-forming toxin activity